{
  "gene_name": "Regulator of G-protein signaling 10",
  "term_label": "Unknown molecular function",
  "term_id": "UNKNOWN:0001",
  "gene_symbol": "RGS10",
  "gene": "UniProtKB:O43665"
}